peptidyl-tRNA hydrolase activity [GO:0004045] (molecular function) Relationships: is a type of GO:0052689; is a type of catalytic activity, acting on a tRNA [GO:0140101] Sources: RHEA:54448 Definition: Catalysis of the reaction: an N-acyl-L-alpha-aminoacyl-tRNA + H2O = an N-acyl-L-amino acid + a tRNA + H+. Also known as: aminoacyl-tRNA hydrolase reaction, D-tyrosyl-tRNA hydrolase activity, N-substituted aminoacyl transfer RNA hydrolase activity, aminoacyl-tRNA aminoacylhydrolase activity, aminoacyl-transfer ribonucleate hydrolase activity